{
  "term_label": "melanosome",
  "gene": "UniProtKB:Q16655",
  "term_id": "GO:0042470",
  "gene_name": "Melanoma antigen recognized by T-cells 1",
  "gene_symbol": "MLANA"
}